{
  "gene_symbol": "IFRD1",
  "term_id": "UNKNOWN:0002",
  "gene": "UniProtKB:O00458",
  "term_label": "Unknown biological process",
  "gene_name": "Interferon-related developmental regulator 1"
}